{
  "gene": "UniProtKB:P05413",
  "gene_symbol": "FABP3",
  "term_id": "GO:0005829",
  "gene_name": "Fatty acid-binding protein, heart",
  "term_label": "cytosol"
}